{
  "gene": "UniProtKB:P52735",
  "term_label": "cytoplasm",
  "gene_name": "Guanine nucleotide exchange factor VAV2",
  "gene_symbol": "VAV2",
  "term_id": "GO:0005737"
}